negative regulation of paraxial mesodermal cell fate specification [GO:0048351] (biological process) Sources: GOC:dgh Also known as: down regulation of paraxial mesodermal cell fate specification, down-regulation of paraxial mesodermal cell fate specification, downregulation of paraxial mesodermal cell fate specification, inhibition of paraxial mesodermal cell fate specification Relationships: is a type of negative regulation of mesodermal cell fate specification [GO:0042662]; is a type of GO:0048349; negatively regulates GO:0048348 Definition: Any process that stops, prevents, or reduces the frequency, rate or extent of paraxial mesoderm cell fate specification.